nor-spermidine metabolic process [GO:0046204] (biological process) Also known as: nor-spermidine metabolism Definition: The chemical reactions and pathways involving nor-spermidine, a compound related to spermidine, N-(3-aminopropyl)-1,4-diaminobutane. Sources: GOC:ai Subtypes: nor-spermidine biosynthetic process [GO:0045312], nor-spermidine catabolic process [GO:0046205] Relationships: is a type of GO:0006595